lateral motor column neuron differentiation [GO:0021525] (biological process) References: PMID:11262869 Sources: GOC:cls, GOC:dgh, GOC:dph, GOC:jid, GO_REF:0000021 Definition: The process in which differentiating motor neurons in the neural tube acquire the specialized structural and/or functional features of lateral motor column neurons. Lateral motor column neurons are generated only on limb levels and send axons into the limb mesenchyme. Differentiation includes the processes involved in commitment of a cell to a specific fate. Relationships: is a type of spinal cord motor neuron differentiation [GO:0021522]; is part of somatic motor neuron differentiation [GO:0021523]